negative regulation of osteoclast proliferation [GO:0090291] (biological process) Relationships: is a type of negative regulation of leukocyte proliferation [GO:0070664]; is_a regulation of osteoclast proliferation [GO:0090289]; negatively regulates osteoclast proliferation [GO:0002158] Sources: GOC:tb Definition: Any process that decreases the rate, frequency, or extent of the multiplication or reproduction of osteoclasts, resulting in the expansion of an osteoclast cell population.